{
  "gene_name": "Zinc finger protein 492",
  "gene": "UniProtKB:Q9P255",
  "term_label": "Unknown cellular component",
  "gene_symbol": "ZNF492",
  "term_id": "UNKNOWN:0003"
}